{
  "gene_symbol": "PATE1",
  "term_id": "UNKNOWN:0002",
  "gene_name": "Prostate and testis expressed protein 1",
  "gene": "UniProtKB:Q8WXA2",
  "term_label": "Unknown biological process"
}